hormone transport [GO:0009914] (biological process) Definition: The directed movement of hormones into, out of or within a cell, or between cells, by means of some agent such as a transporter or pore. Sources: GOC:tb Relationships: is a type of transport [GO:0006810]; is a type of regulation of hormone levels [GO:0010817] Subtypes: cytokinin transport [GO:0010184], hormone secretion [GO:0046879], auxin transport [GO:0060918], thyroid hormone transport [GO:0070327]